{
  "gene_symbol": "COL5A3",
  "term_id": "GO:0030199",
  "gene": "UniProtKB:P25940",
  "term_label": "collagen fibril organization",
  "gene_name": "Collagen alpha-3(V) chain"
}